{
  "term_id": "UNKNOWN:0002",
  "gene_name": "ASNSD1 upstream open reading frame protein",
  "term_label": "Unknown biological process",
  "gene_symbol": "ASDURF",
  "gene": "UniProtKB:L0R819"
}